{
  "gene_name": "Carboxypeptidase B2",
  "term_id": "GO:0005615",
  "term_label": "extracellular space",
  "gene_symbol": "CPB2",
  "gene": "UniProtKB:Q96IY4"
}